{
  "gene_name": "Protein adenylyltransferase FICD",
  "term_id": "GO:0018117",
  "term_label": "protein adenylylation",
  "gene": "UniProtKB:Q9BVA6",
  "gene_symbol": "FICD"
}